positive regulation of lung blood pressure [GO:0061766] (biological process) Definition: The process that increases the force with which blood travels through the lungs. Also known as: positive regulation of pulmonary blood pressure References: PMID:22161164 Sources: GOC:BHF, GOC:BHF_miRNA, GOC:bc Relationships: is a type of regulation of lung blood pressure [GO:0014916]